{
  "term_id": "UNKNOWN:0002",
  "gene_symbol": "GOLGA8G",
  "gene_name": "Putative golgin subfamily A member 8F_8G",
  "gene": "UniProtKB:Q08AF8",
  "term_label": "Unknown biological process"
}